{
  "gene_symbol": "RND1",
  "term_label": "GTP binding",
  "gene_name": "Rho-related GTP-binding protein Rho6",
  "term_id": "GO:0005525",
  "gene": "UniProtKB:Q92730"
}